{
  "term_id": "GO:0046872",
  "gene_symbol": "MT1E",
  "term_label": "metal ion binding",
  "gene_name": "Metallothionein-1E",
  "gene": "UniProtKB:P04732"
}